{
  "gene": "UniProtKB:O75390",
  "term_id": "GO:0006099",
  "gene_symbol": "CS",
  "term_label": "tricarboxylic acid cycle",
  "gene_name": "Citrate synthase, mitochondrial"
}